{
  "term_label": "vesicle-mediated transport",
  "gene_symbol": "TBC1D4",
  "term_id": "GO:0016192",
  "gene": "UniProtKB:O60343",
  "gene_name": "TBC1 domain family member 4"
}